{
  "gene": "UniProtKB:Q96GE4",
  "term_id": "GO:0000922",
  "term_label": "spindle pole",
  "gene_name": "Centrosomal protein of 95 kDa",
  "gene_symbol": "CEP95"
}